regulatory ncRNA processing [GO:0070918] (BP) Definition: A process leading to the generation of a functional regulatory non-coding RNA. References: PMID:15196465, PMID:19239886 Sources: GOC:mah Also known as: gene silencing by RNA, production of guide RNA, gene silencing by RNA, production of small RNA, primary sncRNA processing, production of small RNA involved in gene silencing by RNA, small regulatory ncRNA maturation, small regulatory ncRNA processing, sncRNA processing, sncRNA production Relationships: is a type of RNA processing [GO:0006396]; is part of regulatory ncRNA-mediated gene silencing [GO:0031047] Subtypes: siRNA processing [GO:0030422], GO:0034587, GO:0035196, GO:0043628, tRNA-derived regulatory ncRNA processing [GO:0140891] Regulation: regulated by regulation of regulatory ncRNA processing [GO:0070920]